{
  "term_id": "GO:0005634",
  "gene_symbol": "CLK3",
  "gene": "UniProtKB:P49761",
  "term_label": "nucleus",
  "gene_name": "Dual specificity protein kinase CLK3"
}